valine N-monooxygenase (oxime forming) activity [GO:0102002] (molecular function) Relationships: is a type of oxidoreductase activity, acting on paired donors, with incorporation or reduction of molecular oxygen, NAD(P)H as one donor, and incorporation of one atom of oxygen [GO:0016709] Definition: Catalysis of the reaction: L-valine + 2 O2 + 2 NADPH(4-) + 2 H+ = (E)-2-methylpropanal oxime + 2 NADP(3-) + carbon dioxide + 3 H2O. Sources: EC:1.14.14.38